positive regulation of motor neuron migration [GO:1905485] (biological process) References: PMID:16516839 Sources: GOC:TermGenie, GO_REF:0000058 Subtypes: positive regulation of lateral motor column neuron migration [GO:1902078] Relationships: is a type of GO:1905483; is a type of positive regulation of neuron migration [GO:2001224]; positively regulates motor neuron migration [GO:0097475] Definition: Any process that activates or increases the frequency, rate or extent of motor neuron migration. Also known as: up regulation of motor neuron migration, up-regulation of motor neuron migration, upregulation of motor neuron migration, activation of motor neuron migration